{
  "gene_name": "Proenkephalin-A",
  "gene": "UniProtKB:P01210",
  "term_label": "opioid receptor binding",
  "term_id": "GO:0031628",
  "gene_symbol": "PENK"
}